{
  "gene_name": "Advillin",
  "gene": "UniProtKB:O75366",
  "term_label": "phosphatidylinositol-4,5-bisphosphate binding",
  "term_id": "GO:0005546",
  "gene_symbol": "AVIL"
}